photosynthesis, light harvesting in photosystem I [GO:0009768] (biological process) Definition: After a photon of light is absorbed by one of the many chlorophyll molecules, in one of the light-harvesting complexes of an antenna on photosystem I, some of the absorbed energy is transferred to the pair of chlorophyll molecules in the reaction center. Relationships: is a type of GO:0009765 Sources: GOC:jid, ISBN:0716731363, ISBN:0816017360